lateral plasma membrane [GO:0016328] (cellular component) Sources: GOC:hb, GOC:mah, GOC:pr Definition: The portion of the plasma membrane at the lateral side of the cell. In epithelial cells, lateral plasma membranes are on the sides of cells which lie at the interface of adjacent cells. Relationships: is a type of cellular anatomical structure [GO:0110165]; BFO_0000050 GO:0005886